purine deoxyribonucleotide salvage [GO:0106381] (biological process) Relationships: is a type of purine deoxyribonucleotide biosynthetic process [GO:0009153]; is a type of purine nucleotide salvage [GO:0032261] Definition: Any process which produces a purine deoxyribonucleotide from derivatives of it, without de novo synthesis. References: PMID:6605343 Subtypes: GO:0106383, dGMP salvage [GO:0106384], GO:0106385